{
  "term_id": "GO:0045275",
  "gene": "UniProtKB:P0C7P4",
  "gene_name": "Putative cytochrome b-c1 complex subunit Rieske-like protein 1",
  "term_label": "respiratory chain complex III",
  "gene_symbol": "UQCRFS1P1"
}